{
  "gene_symbol": "CDC14C",
  "term_label": "protein serine/threonine phosphatase activity",
  "gene": "UniProtKB:A4D256",
  "gene_name": "Dual specificity protein phosphatase CDC14C",
  "term_id": "GO:0004722"
}